{
  "gene": "UniProtKB:P62316",
  "term_label": "pICln-Sm protein complex",
  "gene_symbol": "SNRPD2",
  "term_id": "GO:0034715",
  "gene_name": "Small nuclear ribonucleoprotein Sm D2"
}